{
  "term_id": "GO:0005737",
  "gene_symbol": "MYO18A",
  "term_label": "cytoplasm",
  "gene": "UniProtKB:Q92614",
  "gene_name": "Unconventional myosin-XVIIIa"
}